termination of signal transduction [GO:0023021] (biological process) Sources: GOC:mtg_signal Relationships: is a type of negative regulation of signal transduction [GO:0009968] Subtypes: termination of T cell signal transduction [GO:0023022], termination of Roundabout signal transduction [GO:0035554], termination of G protein-coupled receptor signaling pathway [GO:0038032] Note: Note that this term encompasses both the control point when the instruction is given for the process to cease and the actual cessation of the process. A process can persist for some time after that signal that induced the process is withdrawn. Definition: The signaling process in which signal transduction is brought to an end rather than being reversibly modulated.